{
  "term_label": "exonucleolytic trimming to generate mature 3'-end of 5.8S rRNA from tricistronic rRNA transcript (SSU-rRNA, 5.8S rRNA, LSU-rRNA)",
  "term_id": "GO:0000467",
  "gene_symbol": "ERI2",
  "gene_name": "ERI1 exoribonuclease 2",
  "gene": "UniProtKB:A8K979"
}